{
  "gene_symbol": "ALG12",
  "gene_name": "Dol-P-Man:Man(7)GlcNAc(2)-PP-Dol alpha-1,6-mannosyltransferase",
  "term_label": "protein N-linked glycosylation",
  "term_id": "GO:0006487",
  "gene": "UniProtKB:Q9BV10"
}